{
  "gene_symbol": "NAT14",
  "gene_name": "Probable N-acetyltransferase 14",
  "gene": "UniProtKB:Q8WUY8",
  "term_id": "GO:0008080",
  "term_label": "N-acetyltransferase activity"
}